{
  "gene_name": "Transcription factor 20",
  "term_label": "positive regulation of transcription by RNA polymerase II",
  "gene": "UniProtKB:Q9UGU0",
  "term_id": "GO:0045944",
  "gene_symbol": "TCF20"
}